apoptotic process involved in heart valve morphogenesis [GO:0003276] (biological process) Sources: GOC:mtg_apoptosis, GOC:mtg_heart Relationships: is a type of GO:0003278; is part of heart valve morphogenesis [GO:0003179] Definition: Any apoptotic process that contributes to the shaping of a heart valve. Also known as: apoptosis involved in heart valve morphogenesis